regulation of filamentous growth of a population of unicellular organisms in response to starvation [GO:1900434] (biological process) Subtypes: positive regulation of filamentous growth of a population of unicellular organisms in response to starvation [GO:1900436] Definition: Any process that modulates the frequency, rate or extent of filamentous growth of a population of unicellular organisms in response to starvation. Sources: GOC:TermGenie, GOC:di Relationships: is a type of regulation of response to nutrient levels [GO:0032107]; is a type of regulation of response to stress [GO:0080134]; is a type of regulation of filamentous growth of a population of unicellular organisms [GO:1900428]; regulates filamentous growth of a population of unicellular organisms in response to starvation [GO:0036170]